positive regulation of snoRNA processing [GO:1902798] (biological process) Also known as: up regulation of snoRNA processing, up-regulation of snoRNA processing, upregulation of snoRNA processing, activation of snoRNA processing Definition: Any process that activates or increases the frequency, rate or extent of snoRNA processing. References: PMID:24210919 Sources: GOC:TermGenie, GO_REF:0000058 Relationships: is a type of positive regulation of gene expression [GO:0010628]; is a type of GO:1902796; is a type of positive regulation of snoRNA metabolic process [GO:1903325]; positively regulates sno(s)RNA processing [GO:0043144]